{
  "gene_symbol": "ATP1A3",
  "gene": "UniProtKB:P13637",
  "gene_name": "Sodium_potassium-transporting ATPase subunit alpha-3",
  "term_label": "intracellular sodium ion homeostasis",
  "term_id": "GO:0006883"
}